{
  "term_id": "GO:0006998",
  "gene_name": "Myotonin-protein kinase",
  "gene_symbol": "DMPK",
  "term_label": "nuclear envelope organization",
  "gene": "UniProtKB:Q09013"
}